{
  "gene_symbol": "ZNF330",
  "gene": "UniProtKB:Q9Y3S2",
  "term_label": "Unknown molecular function",
  "term_id": "UNKNOWN:0001",
  "gene_name": "Zinc finger protein 330"
}